bacterial biofilm matrix [GO:0097311] (cellular component) References: PMID:22571672 Sources: GOC:imk, Wikipedia:Biofilm Relationships: is a type of biofilm matrix [GO:0062039] Definition: A structure lying external to bacterial cells. A biofilm is an aggregate of surface-associated bacteria, and the biofilm matrix is the envelope of polymeric substances that surrounds the bacteria.